{
  "term_id": "GO:0030425",
  "gene_symbol": "CHRM1",
  "term_label": "dendrite",
  "gene_name": "Muscarinic acetylcholine receptor M1",
  "gene": "UniProtKB:P11229"
}